azole transmembrane transporter activity [GO:1901474] (molecular function) Subtypes: GO:0005290, thiamine transmembrane transporter activity [GO:0015234], fluconazole transmembrane transporter activity [GO:0015244], sulfathiazole transmembrane transporter activity [GO:0015546], GO:0045119, ABC-type azole transporter activity [GO:0140394], histamine transmembrane transporter activity [GO:0160173], aminotriazole transmembrane transporter activity [GO:1901478], GO:1903089, carcinine transmembrane transporter activity [GO:1905131] Sources: GOC:go_curators, ISBN:3527307206, Wikipedia:Azole Definition: Enables the directed movement of azoles, heterocyclic compound found in many biologically important substances, from one side of a membrane to the other. Relationships: is a type of transmembrane transporter activity [GO:0022857]; is part of GO:0045117 Also known as: azole transporter activity